{
  "gene": "UniProtKB:Q9Y446",
  "gene_symbol": "PKP3",
  "term_label": "cadherin binding",
  "gene_name": "Plakophilin-3",
  "term_id": "GO:0045296"
}